{
  "term_id": "GO:0036297",
  "gene": "UniProtKB:Q9H1E3",
  "term_label": "interstrand cross-link repair",
  "gene_name": "Nuclear ubiquitous casein and cyclin-dependent kinase substrate 1",
  "gene_symbol": "NUCKS1"
}